{
  "gene_name": "Multiple epidermal growth factor-like domains protein 9",
  "term_id": "UNKNOWN:0002",
  "gene_symbol": "MEGF9",
  "gene": "UniProtKB:Q9H1U4",
  "term_label": "Unknown biological process"
}